{
  "gene": "UniProtKB:Q9P275",
  "term_label": "cysteine-type deubiquitinase activity",
  "term_id": "GO:0004843",
  "gene_symbol": "USP36",
  "gene_name": "Ubiquitin carboxyl-terminal hydrolase 36"
}